{
  "gene_name": "Zinc finger protein 232",
  "gene_symbol": "ZNF232",
  "term_label": "DNA-binding transcription factor activity, RNA polymerase II-specific",
  "gene": "UniProtKB:Q9UNY5",
  "term_id": "GO:0000981"
}